negative regulation of monocyte differentiation [GO:0045656] (biological process) Relationships: is a type of negative regulation of myeloid leukocyte differentiation [GO:0002762]; is a type of regulation of monocyte differentiation [GO:0045655]; RO_0002212 GO:0030224 Also known as: down regulation of monocyte differentiation, down-regulation of monocyte differentiation, downregulation of monocyte differentiation, inhibition of monocyte differentiation Sources: GOC:go_curators Definition: Any process that stops, prevents, or reduces the frequency, rate or extent of monocyte differentiation.